non-classical arabinogalactan protein metabolic process [GO:0010407] (biological process) Definition: The chemical reactions and pathways involving a cell wall arabinogalactan II glycoprotein where other amino acids besides Hyp, Ala, Ser, Thr and Gly can be present and grouped into regions, such as a Cys-rich or Asn-rich domains. Sources: GOC:tair_curators Also known as: non-classical arabinogalactan protein metabolism Relationships: is a type of GO:0010405